{
  "term_label": "Unknown biological process",
  "gene_symbol": "SUB1",
  "gene_name": "Activated RNA polymerase II transcriptional coactivator p15",
  "term_id": "UNKNOWN:0002",
  "gene": "UniProtKB:P53999"
}